{
  "gene_symbol": "LCP1",
  "gene": "UniProtKB:P13796",
  "gene_name": "Plastin-2",
  "term_label": "actin filament bundle assembly",
  "term_id": "GO:0051017"
}